pattern specification process [GO:0007389] (biological process) Sources: GOC:go_curators, GOC:isa_complete, ISBN:0521436125 Definition: Any developmental process that results in the creation of defined areas or spaces within an organism to which cells respond and eventually are instructed to differentiate. Also known as: pattern biosynthesis, pattern formation Relationships: is a type of multicellular organismal process [GO:0032501]; is part of multicellular organism development [GO:0007275] Subtypes: GO:0003002, segment specification [GO:0007379], axis specification [GO:0009798], specification of symmetry [GO:0009799], embryonic pattern specification [GO:0009880], GO:0016318, GO:0035161, GO:0035287, regulation of R8 cell spacing in compound eye [GO:0045468], GO:0060432, GO:0060896, GO:0061004, maintenance of left/right asymmetry [GO:0061968], GO:0065001, renal system pattern specification [GO:0072048], GO:0080006